{
  "gene": "UniProtKB:P21506",
  "term_id": "GO:0000977",
  "gene_name": "Zinc finger protein 10",
  "term_label": "RNA polymerase II transcription regulatory region sequence-specific DNA binding",
  "gene_symbol": "ZNF10"
}